{
  "term_id": "GO:0006089",
  "term_label": "lactate metabolic process",
  "gene_symbol": "LDHAL6B",
  "gene": "UniProtKB:Q9BYZ2",
  "gene_name": "L-lactate dehydrogenase A-like 6B"
}